regulation of slow-twitch skeletal muscle fiber contraction [GO:0031449] (biological process) Definition: Any process that modulates the frequency, rate or extent of slow-twitch skeletal muscle contraction. Sources: GOC:dph, GOC:ef, GOC:mah, GOC:mtg_muscle, GOC:tb Also known as: regulation of slow-twitch skeletal muscle contraction Relationships: is a type of regulation of twitch skeletal muscle contraction [GO:0014724]; regulates slow-twitch skeletal muscle fiber contraction [GO:0031444] Subtypes: negative regulation of slow-twitch skeletal muscle fiber contraction [GO:0031450], positive regulation of slow-twitch skeletal muscle fiber contraction [GO:0031451]